{
  "term_label": "toll-like receptor signaling pathway",
  "gene": "UniProtKB:Q9Y2C9",
  "gene_name": "Toll-like receptor 6",
  "term_id": "GO:0002224",
  "gene_symbol": "TLR6"
}